{
  "term_id": "UNKNOWN:0003",
  "term_label": "Unknown cellular component",
  "gene_name": "Serine_threonine-protein kinase 38-like",
  "gene_symbol": "STK38L",
  "gene": "UniProtKB:Q9Y2H1"
}